{
  "gene_symbol": "CNOT3",
  "gene": "UniProtKB:O75175",
  "gene_name": "CCR4-NOT transcription complex subunit 3",
  "term_id": "GO:0030015",
  "term_label": "CCR4-NOT core complex"
}